{
  "term_label": "SREBP-SCAP complex",
  "gene_symbol": "SCAP",
  "term_id": "GO:0032936",
  "gene_name": "Sterol regulatory element-binding protein cleavage-activating protein",
  "gene": "UniProtKB:Q12770"
}